Dxr protein complex [GO:1990065] (cellular component) Definition: A protein complex that is involved in the MEP pathway of IPP biosynthesis. It catalyzes the NADP-dependent rearrangement and reduction of 1-deoxy-D-xylulose-5-phosphate (DXP) to 2-C-methyl-D-erythritol 4-phosphate (MEP). References: PMID:15339150 Sources: GOC:bhm Relationships: is a type of protein-containing complex [GO:0032991] Also known as: 1-deoxy-D-xylulose 5-phosphate reductoisomerase complex